{
  "term_id": "GO:0003677",
  "gene_symbol": "TIGD3",
  "gene": "UniProtKB:Q6B0B8",
  "term_label": "DNA binding",
  "gene_name": "Tigger transposable element-derived protein 3"
}